{
  "term_label": "NAD transmembrane transporter activity",
  "term_id": "GO:0051724",
  "gene": "UniProtKB:Q3SY17",
  "gene_name": "Mitochondrial nicotinamide adenine dinucleotide transporter SLC25A52",
  "gene_symbol": "SLC25A52"
}